{
  "gene": "UniProtKB:Q8NCQ5",
  "gene_name": "F-box only protein 15",
  "term_id": "GO:0019005",
  "gene_symbol": "FBXO15",
  "term_label": "SCF ubiquitin ligase complex"
}